{
  "gene": "UniProtKB:P08133",
  "gene_symbol": "ANXA6",
  "term_id": "GO:0005544",
  "gene_name": "Annexin A6",
  "term_label": "calcium-dependent phospholipid binding"
}